{
  "gene_name": "Uncharacterized protein C5orf67",
  "term_label": "Unknown cellular component",
  "term_id": "UNKNOWN:0003",
  "gene_symbol": "C5orf67",
  "gene": "UniProtKB:F2Z3F1"
}